sodium ion-transporting F-type ATPase complex [GO:0016473] (cellular component) Also known as: sodium-translocating F-type ATPase complex Definition: A sodium ion-transporting two-sector ATPase complex that catalyzes the phosphorylation of ADP to ATP. The complex comprises a membrane sector (F0) that carries out proton transport and a cytoplasmic compartment sector (F1) that catalyzes ATP synthesis by a rotational mechanism. References: PMID:14656431 Sources: GOC:mah Relationships: is_a GO:0016472